{
  "gene_name": "Integrin alpha-X",
  "term_label": "cell surface",
  "term_id": "GO:0009986",
  "gene_symbol": "ITGAX",
  "gene": "UniProtKB:P20702"
}